{
  "term_label": "Unknown cellular component",
  "gene_name": "Ras association domain-containing protein 8",
  "gene_symbol": "RASSF8",
  "term_id": "UNKNOWN:0003",
  "gene": "UniProtKB:Q8NHQ8"
}